{
  "gene_name": "Protein TANC1",
  "term_id": "GO:0098978",
  "gene": "UniProtKB:Q9C0D5",
  "term_label": "glutamatergic synapse",
  "gene_symbol": "TANC1"
}